positive regulation of ethanol catabolic process [GO:1900066] (biological process) Definition: Any process that activates or increases the frequency, rate or extent of ethanol catabolic process. Also known as: positive regulation of ethanol breakdown, positive regulation of ethanol catabolism, positive regulation of ethanol degradation, up regulation of ethanol breakdown, up regulation of ethanol catabolism, up regulation of ethanol degradation, up-regulation of ethanol breakdown, up-regulation of ethanol catabolism, up-regulation of ethanol degradation, upregulation of ethanol breakdown, upregulation of ethanol catabolism, upregulation of ethanol degradation, activation of ethanol breakdown, activation of ethanol catabolic process, activation of ethanol catabolism, activation of ethanol degradation, up regulation of ethanol catabolic process, up-regulation of ethanol catabolic process, upregulation of ethanol catabolic process References: PMID:10608811, PMID:7760841 Sources: GOC:TermGenie Relationships: is a type of GO:1900065; is a type of positive regulation of alcohol catabolic process [GO:1900421]; positively regulates ethanol catabolic process [GO:0006068]